{
  "term_id": "GO:0030280",
  "gene": "UniProtKB:P02538",
  "gene_symbol": "KRT6A",
  "term_label": "structural constituent of skin epidermis",
  "gene_name": "Keratin, type II cytoskeletal 6A"
}